{
  "gene_name": "NADH dehydrogenase [ubiquinone] iron-sulfur protein 4, mitochondrial",
  "term_label": "respiratory chain complex I",
  "term_id": "GO:0045271",
  "gene_symbol": "NDUFS4",
  "gene": "UniProtKB:O43181"
}